{
  "term_id": "GO:0005886",
  "gene": "UniProtKB:Q13393",
  "gene_name": "Phospholipase D1",
  "term_label": "plasma membrane",
  "gene_symbol": "PLD1"
}